positive regulation of mitotic cytokinesis [GO:1903490] (biological process) Also known as: positive regulation of cytokinesis after mitosis, up regulation of cytokinesis after mitosis, up regulation of mitotic cytokinesis, up-regulation of cytokinesis after mitosis, up-regulation of mitotic cytokinesis, upregulation of cytokinesis after mitosis, upregulation of mitotic cytokinesis, activation of cytokinesis after mitosis, activation of mitotic cytokinesis Definition: Any process that activates or increases the frequency, rate or extent of mitotic cytokinesis. References: PMID:24920823 Sources: GOC:TermGenie, GO_REF:0000058 Subtypes: GO:1903438 Relationships: is_a positive regulation of cytokinesis [GO:0032467]; is a type of regulation of mitotic cytokinesis [GO:1902412]; positively regulates GO:0000281